chromoplast membrane [GO:0046862] (cellular component) Sources: GOC:ai, GOC:mah Subtypes: chromoplast inner membrane [GO:0031899], GO:0031900 Relationships: is a type of plastid membrane [GO:0042170]; is part of chromoplast envelope [GO:0031898] Definition: Either of the lipid bilayers that surround a chromoplast and form the chromoplast envelope.